{
  "gene_symbol": "MCM3",
  "gene": "UniProtKB:P25205",
  "term_label": "nucleus",
  "gene_name": "DNA replication licensing factor MCM3",
  "term_id": "GO:0005634"
}